{
  "term_id": "GO:0051402",
  "gene": "UniProtKB:Q00535",
  "gene_name": "Cyclin-dependent kinase 5",
  "gene_symbol": "CDK5",
  "term_label": "neuron apoptotic process"
}